{
  "term_id": "UNKNOWN:0002",
  "gene_symbol": "CXorf51B",
  "gene_name": "Uncharacterized protein CXorf51B",
  "term_label": "Unknown biological process",
  "gene": "UniProtKB:P0DPH9"
}